{
  "term_id": "GO:0012505",
  "gene_symbol": "RNF145",
  "term_label": "endomembrane system",
  "gene": "UniProtKB:Q96MT1",
  "gene_name": "RING finger protein 145"
}